{
  "term_id": "GO:0015459",
  "gene_symbol": "KCNV1",
  "gene": "UniProtKB:Q6PIU1",
  "term_label": "potassium channel regulator activity",
  "gene_name": "Potassium voltage-gated channel subfamily V member 1"
}